{
  "gene": "UniProtKB:Q49AS3",
  "gene_symbol": "LRRC37A5P",
  "gene_name": "Putative protein LRRC37A5P",
  "term_label": "Unknown molecular function",
  "term_id": "UNKNOWN:0001"
}